{
  "term_label": "Unknown molecular function",
  "term_id": "UNKNOWN:0001",
  "gene_name": "Retinoblastoma-binding protein 5",
  "gene": "UniProtKB:Q15291",
  "gene_symbol": "RBBP5"
}